{
  "gene": "UniProtKB:P40425",
  "gene_name": "Pre-B-cell leukemia transcription factor 2",
  "term_label": "RNA polymerase II cis-regulatory region sequence-specific DNA binding",
  "term_id": "GO:0000978",
  "gene_symbol": "PBX2"
}